pullulan catabolic process [GO:0051678] (biological process) Definition: The chemical reactions and pathways resulting in the breakdown of pullulan, a neutral linear polysaccharide composed of repeating units of maltotriose joined by alpha-(1,6)-linkages. Sources: GOC:ai Relationships: is a type of glucan catabolic process [GO:0009251]; is a type of pullulan metabolic process [GO:0051676]